{
  "gene_symbol": "CLMN",
  "gene": "UniProtKB:Q96JQ2",
  "gene_name": "Calmin",
  "term_id": "GO:0008285",
  "term_label": "negative regulation of cell population proliferation"
}